{
  "gene_symbol": "ATG2A",
  "gene": "UniProtKB:Q2TAZ0",
  "gene_name": "Autophagy-related protein 2 homolog A",
  "term_label": "reticulophagy",
  "term_id": "GO:0061709"
}